{
  "gene_name": "Stereocilin",
  "term_id": "GO:0007160",
  "gene": "UniProtKB:Q7RTU9",
  "term_label": "cell-matrix adhesion",
  "gene_symbol": "STRC"
}